{
  "term_id": "GO:0005737",
  "gene_name": "Glycogen synthase kinase-3 alpha",
  "gene_symbol": "GSK3A",
  "gene": "UniProtKB:P49840",
  "term_label": "cytoplasm"
}